negative regulation of thymocyte migration [GO:2000411] (biological process) Sources: GOC:mah Relationships: is a type of negative regulation of T cell migration [GO:2000405]; is a type of GO:2000410; negatively regulates thymocyte migration [GO:0072679] Also known as: negative regulation of thymic lymphocyte migration, negative regulation of immature T cell migration, negative regulation of immature T lymphocyte migration, negative regulation of immature T-cell migration, negative regulation of immature T-lymphocyte migration Definition: Any process that stops, prevents or reduces the frequency, rate or extent of thymocyte migration. Subtypes: GO:2000414